{
  "gene_symbol": "TLR9",
  "term_id": "GO:0005886",
  "gene": "UniProtKB:Q9NR96",
  "term_label": "plasma membrane",
  "gene_name": "Toll-like receptor 9"
}